{
  "gene_symbol": "S100A10",
  "gene": "UniProtKB:P60903",
  "term_id": "GO:0044325",
  "gene_name": "Protein S100-A10",
  "term_label": "transmembrane transporter binding"
}